{
  "term_id": "UNKNOWN:0002",
  "gene": "UniProtKB:Q8NBM4",
  "gene_symbol": "UBAC2",
  "term_label": "Unknown biological process",
  "gene_name": "Ubiquitin-associated domain-containing protein 2"
}